trichloroethylene catabolic process [GO:0050696] (biological process) Sources: GOC:ai Also known as: trichloroethene catabolic process, trichloroethene catabolism, trichloroethylene breakdown, trichloroethylene catabolism, trichloroethylene degradation Relationships: is a type of trichloroethylene metabolic process [GO:0018979]; is a type of GO:0042205 Definition: The chemical reactions and pathways resulting in the breakdown of trichloroethylene, a toxic, colorless, photoreactive, chlorinated hydrocarbon liquid, commonly used as a metal degreaser and solvent.